{
  "term_label": "Unknown molecular function",
  "gene_symbol": "ADGB",
  "gene": "UniProtKB:Q8N7X0",
  "term_id": "UNKNOWN:0001",
  "gene_name": "Androglobin"
}